mesonephric tubule morphogenesis [GO:0072171] (biological process) Sources: GOC:mtg_kidney_jan10 Subtypes: ureteric bud morphogenesis [GO:0060675], mesonephric nephron tubule morphogenesis [GO:0061240], mesonephric duct morphogenesis [GO:0072180] Definition: The process in which the anatomical structures of a mesonephric tubule are generated and organized. A mesonephric tubule is an epithelial tube that is part of the mesonephros. Relationships: is a type of nephron tubule morphogenesis [GO:0072078]; is part of mesonephric tubule development [GO:0072164]